{
  "gene": "UniProtKB:Q5VWT5",
  "term_label": "T cell receptor signaling pathway",
  "gene_name": "FYN-binding protein 2",
  "gene_symbol": "FYB2",
  "term_id": "GO:0050852"
}